regulation of polyamine transmembrane transport [GO:1902267] (biological process) Subtypes: negative regulation of polyamine transmembrane transport [GO:1902268], positive regulation of polyamine transmembrane transport [GO:1902269] Definition: Any process that modulates the frequency, rate or extent of polyamine transmembrane transport. Relationships: is_a GO:0034762; regulates polyamine transmembrane transport [GO:1902047] References: PMID:23755272 Sources: GOC:TermGenie